{
  "gene": "UniProtKB:Q9NY72",
  "term_id": "GO:0086091",
  "term_label": "regulation of heart rate by cardiac conduction",
  "gene_name": "Sodium channel subunit beta-3",
  "gene_symbol": "SCN3B"
}